{
  "gene_symbol": "ZFYVE1",
  "gene_name": "Zinc finger FYVE domain-containing protein 1",
  "term_id": "GO:0032266",
  "gene": "UniProtKB:Q9HBF4",
  "term_label": "phosphatidylinositol-3-phosphate binding"
}